{
  "gene_symbol": "ACSBG2",
  "term_id": "GO:0005737",
  "gene": "UniProtKB:Q5FVE4",
  "gene_name": "Long-chain-fatty-acid--CoA ligase ACSBG2",
  "term_label": "cytoplasm"
}